negative regulation of microvillus assembly [GO:1903697] (biological process) Also known as: down regulation of microvillus assembly, down-regulation of microvillus assembly, downregulation of microvillus assembly, inhibition of microvillus assembly, down regulation of microvillus biogenesis, down-regulation of microvillus biogenesis, downregulation of microvillus biogenesis, inhibition of microvillus biogenesis, negative regulation of microvillus biogenesis Relationships: is a type of regulation of microvillus assembly [GO:0032534]; is a type of negative regulation of plasma membrane bounded cell projection assembly [GO:0120033]; negatively regulates microvillus assembly [GO:0030033] Definition: Any process that stops, prevents or reduces the frequency, rate or extent of microvillus assembly. References: PMID:22797597 Sources: GOC:TermGenie, GOC:als, GO_REF:0000058